axonemal microtubule doublet inner sheath [GO:0160110] (cellular component) References: PMID:29430673, PMID:37295417 Sources: GOC:krc Definition: A structural network of microtubule inner proteins (MIPs) located inside the lumens of the A and B tubules of the axonemal microtuble doublet that helps stabilize the doublet microtubule. Relationships: is a type of cellular anatomical structure [GO:0110165]; is part of axonemal doublet microtubule [GO:0097545]